{
  "term_id": "GO:0005886",
  "term_label": "plasma membrane",
  "gene_symbol": "GPR32P1",
  "gene_name": "Putative G-protein coupled receptor GPR32P1",
  "gene": "UniProtKB:Q8NGA4"
}